{
  "term_label": "nucleus",
  "gene_name": "Zinc finger protein 705A",
  "gene": "UniProtKB:Q6ZN79",
  "gene_symbol": "ZNF705A",
  "term_id": "GO:0005634"
}